{
  "gene_symbol": "RAET1G",
  "gene": "UniProtKB:Q6H3X3",
  "gene_name": "UL-16 binding protein 5",
  "term_id": "GO:0002476",
  "term_label": "antigen processing and presentation of endogenous peptide antigen via MHC class Ib"
}